{
  "term_id": "GO:0043565",
  "gene_symbol": "ZNF672",
  "term_label": "sequence-specific DNA binding",
  "gene": "UniProtKB:Q499Z4",
  "gene_name": "Zinc finger protein 672"
}